{
  "term_id": "UNKNOWN:0002",
  "term_label": "Unknown biological process",
  "gene_symbol": "IGSF10",
  "gene_name": "Immunoglobulin superfamily member 10",
  "gene": "UniProtKB:Q6WRI0"
}